regulation of tetrapyrrole biosynthetic process from glutamate [GO:1901410] (biological process) Sources: GOC:TermGenie, GOC:mengo_curators Definition: Any process that modulates the frequency, rate or extent of tetrapyrrole biosynthetic process from glutamate. Relationships: is a type of regulation of tetrapyrrole biosynthetic process [GO:1901463]; is a type of regulation of glutamate metabolic process [GO:2000211]; regulates tetrapyrrole biosynthetic process from glutamate [GO:0033526] Subtypes: negative regulation of tetrapyrrole biosynthetic process from glutamate [GO:1901411], GO:1901412 Also known as: regulation of tetrapyrrole anabolism from glutamate, regulation of tetrapyrrole biosynthesis from glutamate, regulation of tetrapyrrole formation from glutamate, regulation of tetrapyrrole synthesis from glutamate